{
  "term_label": "SUMO binding",
  "term_id": "GO:0032183",
  "gene": "UniProtKB:Q9UHP3",
  "gene_name": "Ubiquitin carboxyl-terminal hydrolase 25",
  "gene_symbol": "USP25"
}